metal chelating activity [GO:0046911] (molecular function) Relationships: is a type of metal ion binding [GO:0046872] Sources: ISBN:0198506732, ISBN:0716731363 Also known as: metal chelation, heavy metal chelation Definition: The formation of bonds from two or more atoms within the same ligand to a metal atom in complexes in which the metal is part of a ring.